{
  "term_id": "GO:0003755",
  "gene_name": "Peptidyl-prolyl cis-trans isomerase FKBP10",
  "gene": "UniProtKB:Q96AY3",
  "gene_symbol": "FKBP10",
  "term_label": "peptidyl-prolyl cis-trans isomerase activity"
}